{
  "gene_symbol": "FMNL2",
  "gene": "UniProtKB:Q96PY5",
  "gene_name": "Formin-like protein 2",
  "term_label": "actin filament binding",
  "term_id": "GO:0051015"
}